{
  "term_id": "UNKNOWN:0001",
  "gene_symbol": "DEPP1",
  "gene_name": "Protein DEPP1",
  "gene": "UniProtKB:Q9NTK1",
  "term_label": "Unknown molecular function"
}